{
  "term_id": "GO:0004843",
  "gene_name": "OTU domain-containing protein 7A",
  "gene_symbol": "OTUD7A",
  "gene": "UniProtKB:Q8TE49",
  "term_label": "cysteine-type deubiquitinase activity"
}